5-dehydro-4-deoxyglucarate dehydratase activity [GO:0047448] (molecular function) Definition: Catalysis of the reaction: 5-dehydro-4-deoxy-D-glucarate + H+ = 2,5-dioxopentanoate + CO2 + H2O. Sources: EC:4.2.1.41, RHEA:24608 Also known as: 5-dehydro-4-deoxy-D-glucarate hydro-lyase (decarboxylating), 5-dehydro-4-deoxy-D-glucarate hydro-lyase (decarboxylating; 2,5-dioxopentanoate-forming), 5-keto-4-deoxy-glucarate dehydratase activity, D-4-deoxy-5-ketoglucarate hydro-lyase activity, deoxyketoglucarate dehydratase activity Relationships: is a type of hydro-lyase activity [GO:0016836]